{
  "gene_symbol": "FZD10",
  "gene": "UniProtKB:Q9ULW2",
  "term_label": "Wnt-protein binding",
  "gene_name": "Frizzled-10",
  "term_id": "GO:0017147"
}